{
  "gene": "UniProtKB:Q8TAA1",
  "gene_symbol": "RNASE11",
  "term_label": "Unknown molecular function",
  "gene_name": "Probable ribonuclease 11",
  "term_id": "UNKNOWN:0001"
}